{
  "term_id": "GO:0009986",
  "gene": "UniProtKB:P40198",
  "gene_name": "Carcinoembryonic antigen-related cell adhesion molecule 3",
  "term_label": "cell surface",
  "gene_symbol": "CEACAM3"
}